{
  "gene_symbol": "MTSS1",
  "term_label": "phospholipid binding",
  "term_id": "GO:0005543",
  "gene": "UniProtKB:O43312",
  "gene_name": "Protein MTSS 1"
}